posterior lateral line system development [GO:0048915] (biological process) Relationships: is a type of lateral line system development [GO:0048925]; is part of mechanosensory lateral line system development [GO:0048881] Also known as: PLL References: PMID:15018940 Sources: ISBN:0125296509 Definition: The process whose specific outcome is the progression of the posterior lateral line system over time, from its formation to the mature structure. The posterior lateral line system develops from cranial ectodermal placodes, situated behind the ear, that give rise to both the neuromasts and the posterior lateral line sensory nerves that innervate the neuromasts. The posterior lateral line system consists of small sensory patches (neuromasts) located superficially on the skin or just under the skin in fluid-filled canals on the head of all fishes and most amphibians. The neuromasts are innervated by several lateral line nerves, which project primarily to the hindbrain. The posterior mechanosensory lateral line system is stimulated by local water displacements and vibrations, and detects propulsion of the fish through the water, as well as facilitating shoaling, prey capture, and predator and obstacle avoidance.